{
  "gene_name": "Platelet-activating factor acetylhydrolase IB subunit beta",
  "term_label": "nuclear envelope",
  "gene_symbol": "PAFAH1B1",
  "gene": "UniProtKB:P43034",
  "term_id": "GO:0005635"
}